{
  "term_label": "ceramide catabolic process",
  "gene": "UniProtKB:P19835",
  "gene_name": "Bile salt-activated lipase",
  "gene_symbol": "CEL",
  "term_id": "GO:0046514"
}